outer kinetochore [GO:0000940] (cellular component) Also known as: condensed chromosome outer kinetochore, condensed nuclear chromosome outer kinetochore, outer kinetochore of condensed chromosome, outer kinetochore of condensed nuclear chromosome, outer kinetochore plate References: PMID:11483983 Sources: GOC:clt Relationships: is a type of protein-containing complex [GO:0032991]; is part of GO:0000776 Subtypes: GO:0000444 Definition: The region of a kinetochore most external to centromeric DNA; this outer region mediates kinetochore-microtubule interactions.